(-)-microperfuranone catabolic process [GO:1901511] (biological process) Sources: GOC:TermGenie, GOC:di Definition: The chemical reactions and pathways resulting in the breakdown of (-)-microperfuranone. Also known as: (-)-microperfuranone breakdown, (-)-microperfuranone catabolism, (-)-microperfuranone degradation Relationships: is a type of lactone catabolic process [GO:1901335]; is a type of GO:1901502